{
  "term_label": "calcium-independent cell-cell adhesion",
  "gene_name": "Claudin-2",
  "gene_symbol": "CLDN2",
  "gene": "UniProtKB:P57739",
  "term_id": "GO:0016338"
}